{
  "gene": "UniProtKB:Q5TFG8",
  "term_label": "Unknown molecular function",
  "term_id": "UNKNOWN:0001",
  "gene_symbol": "ZC2HC1B",
  "gene_name": "Zinc finger C2HC domain-containing protein 1B"
}